{
  "gene": "UniProtKB:Q13303",
  "term_id": "GO:0008076",
  "gene_name": "Voltage-gated potassium channel subunit beta-2",
  "term_label": "voltage-gated potassium channel complex",
  "gene_symbol": "KCNAB2"
}